{
  "term_id": "GO:0004879",
  "gene": "UniProtKB:P08235",
  "term_label": "nuclear receptor activity",
  "gene_name": "Mineralocorticoid receptor",
  "gene_symbol": "NR3C2"
}